{
  "gene_name": "Dihydrolipoyllysine-residue succinyltransferase component of 2-oxoglutarate dehydrogenase complex, mitochondrial",
  "term_label": "tricarboxylic acid cycle",
  "gene": "UniProtKB:P36957",
  "term_id": "GO:0006099",
  "gene_symbol": "DLST"
}